regulation of cardiac chamber formation [GO:1901210] (biological process) Also known as: regulation of heart chamber formation Sources: GOC:BHF, GOC:TermGenie Subtypes: negative regulation of cardiac chamber formation [GO:1901211], positive regulation of cardiac chamber formation [GO:1901212], GO:1904942 Relationships: is a type of GO:0050793; regulates GO:0003207 Definition: Any process that modulates the frequency, rate or extent of cardiac chamber formation.